entry of viral genome into host nucleus via retainment of capsid in nuclear pore complex and release of genome into nucleoplasm [GO:0075508] (biological process) Definition: Viral penetration into the host nucleus where a viral capsid enters the host nuclear pore complex (NPC) but remains attached to the pore on the nuclear side. The capsid then disassembles, releasing the viral genome into the nucleoplasm. Note: This mechanism is used by viruses such as Hepadnaviridae whose capsids enter the NPC but are too big to pass intact into the nucleus. References: PMID:22929056 Sources: VZ:989 Relationships: is a type of viral penetration into host nucleus [GO:0075732] Also known as: entry of viral genome into host nucleus via attachment of capsid to nuclear pore complex and release of genome into nucleoplasm